negative regulation of cellular response to drug [GO:2001039] (biological process) Definition: Any process that stops, prevents or reduces the frequency, rate or extent of cellular response to drug. Sources: GOC:obol Relationships: is a type of GO:0048523; is a type of GO:2001024; is a type of GO:2001038; negatively regulates GO:0071466